{
  "gene_symbol": "POU6F2",
  "term_id": "GO:0000981",
  "gene": "UniProtKB:P78424",
  "term_label": "DNA-binding transcription factor activity, RNA polymerase II-specific",
  "gene_name": "POU domain, class 6, transcription factor 2"
}